{
  "term_label": "positive regulation of smooth muscle contraction",
  "gene_name": "Neuromedin-U",
  "gene": "UniProtKB:P48645",
  "gene_symbol": "NMU",
  "term_id": "GO:0045987"
}